{
  "term_id": "UNKNOWN:0003",
  "term_label": "Unknown cellular component",
  "gene_symbol": "PDE8A",
  "gene": "UniProtKB:O60658",
  "gene_name": "High affinity cAMP-specific and IBMX-insensitive 3',5'-cyclic phosphodiesterase 8A"
}